{
  "gene_name": "Gamma-crystallin C",
  "gene": "UniProtKB:P07315",
  "gene_symbol": "CRYGC",
  "term_id": "GO:0005212",
  "term_label": "structural constituent of eye lens"
}